{
  "term_id": "UNKNOWN:0001",
  "gene_name": "Protein NipSnap homolog 1",
  "gene_symbol": "NIPSNAP1",
  "gene": "UniProtKB:Q9BPW8",
  "term_label": "Unknown molecular function"
}